{
  "gene_symbol": "AMN1",
  "gene": "UniProtKB:Q8IY45",
  "term_label": "SCF-dependent proteasomal ubiquitin-dependent protein catabolic process",
  "gene_name": "Protein AMN1 homolog",
  "term_id": "GO:0031146"
}